tagaturonate reductase activity [GO:0009026] (molecular function) Sources: EC:1.1.1.58, RHEA:17813 Also known as: D-altronate:NAD+ 3-oxidoreductase activity, D-tagaturonate reductase activity, TagUAR, altronate dehydrogenase activity, altronate oxidoreductase activity, altronic oxidoreductase activity, tagaturonate dehydrogenase activity Definition: Catalysis of the reaction: D-altronate + NAD+ = D-tagaturonate + H+ + NADH. Relationships: is a type of oxidoreductase activity, acting on the CH-OH group of donors, NAD or NADP as acceptor [GO:0016616]